{
  "gene": "UniProtKB:P05549",
  "gene_symbol": "TFAP2A",
  "gene_name": "Transcription factor AP-2-alpha",
  "term_label": "skeletal system development",
  "term_id": "GO:0001501"
}